regulation of cellotriose catabolic process [GO:2000936] (biological process) Definition: Any process that modulates the frequency, rate or extent of cellotriose catabolic process. Sources: GOC:mengo_curators Also known as: regulation of cellotriose catabolism Relationships: is a type of regulation of carbohydrate catabolic process [GO:0043470]; regulates cellotriose catabolic process [GO:2000894] Subtypes: negative regulation of cellotriose catabolic process [GO:2000937], positive regulation of cellotriose catabolic process [GO:2000938]